{
  "gene_name": "Methionyl-tRNA formyltransferase, mitochondrial",
  "gene_symbol": "MTFMT",
  "term_label": "conversion of methionyl-tRNA to N-formyl-methionyl-tRNA",
  "term_id": "GO:0071951",
  "gene": "UniProtKB:Q96DP5"
}